ABC-type phytochelatin transporter activity [GO:0044604] (molecular function) References: PMID:1396551 Sources: GOC:mah Definition: Enables the directed movement of a phytochelatin from one side of a membrane to the other. Phytochelatins are a group of peptides that bind metals (Cd, Zn, Cu, Pb, Hg) in thiolate coordination complexes. Also known as: ABC-type phytochelatin transmembrane transporter activity, ATP-dependent phytochelatin transmembrane transporter activity, ATPase-coupled phytochelatin transmembrane transporter activity, cadystin transmembrane transporter ATPase activity, cadystin transmembrane transporter activity, cadystin transporter activity, phytochelatin transmembrane transporter ATPase activity, phytochelatin transmembrane transporter activity, phytochelatin transporter activity Relationships: is a type of amide transmembrane transporter activity [GO:0042887]; is a type of ABC-type transporter activity [GO:0140359]; is part of detoxification of inorganic compound [GO:0061687]; is part of phytochelatin transmembrane transport [GO:0071994]